{
  "term_id": "GO:0000395",
  "gene_symbol": "SFSWAP",
  "term_label": "mRNA 5'-splice site recognition",
  "gene_name": "Splicing factor, suppressor of white-apricot homolog",
  "gene": "UniProtKB:Q12872"
}